ATAC complex [GO:0140672] (cellular component) References: PMID:19936620, PMID:20562830, PMID:28966424 Sources: GOC:bhm Also known as: ADA2A-containing complex, Ada Two-A containing complex, Ada two A containing complex, Ada-Two-A-containing complex, G-ATAC complex, KAT2A-containing ATAC complex, KAT2B-containing ATAC complex Definition: A chromatin remodeling complex that regulates transcription via acetylation primarily of nucleosomal histones H3 and possibly H4. Shares the histone acetylation (HAT) module of GCN5/PCAF-ADA2-ADA3-SGF29 (or orthologs) with the related SAGA complex (GO:0000124). Contains HAT subunits GCN5 or PCAF in a mutually exclusive manner. In addition to the HAT module contains DR1/NC2B, KAT14, MBIP, WDR5, YEATS2 and ZZZ3 or orthologs. Also regulates the activity of non-histone targets and orchestrates mitotic progression by regulating Cyclin A degradation through acetylation. Relationships: is a type of GO:0070461